melanin catabolic process [GO:0046150] (biological process) Sources: ISBN:0198506732 Also known as: melanin breakdown, melanin catabolism, melanin degradation Definition: The chemical reactions and pathways resulting in the breakdown of melanins, pigments largely of animal origin. High molecular weight polymers of indole quinone, they are irregular polymeric structures and are divided into three groups: allomelanins in the plant kingdom and eumelanins and phaeomelanins in the animal kingdom. Relationships: is a type of melanin metabolic process [GO:0006582]; is a type of phenol-containing compound catabolic process [GO:0019336]; is a type of pigment catabolic process [GO:0046149]